mitotic sister chromatid cohesion, centromeric [GO:0071962] (biological process) Also known as: centromeric mitotic sister chromatin cohesion, mitotic sister chromatid cohesion at centromere, sister chromatid cohesion at centromere at mitosis Sources: GOC:mah Definition: The cell cycle process in which centromeres of sister chromatids are joined during mitosis. Relationships: is a type of GO:0007064; is a type of centromeric sister chromatid cohesion [GO:0070601]